{
  "gene": "UniProtKB:P45973",
  "term_id": "GO:0005721",
  "gene_name": "Chromobox protein homolog 5",
  "term_label": "pericentric heterochromatin",
  "gene_symbol": "CBX5"
}